{
  "gene_symbol": "WHRN",
  "term_id": "GO:0005929",
  "gene": "UniProtKB:Q9P202",
  "term_label": "cilium",
  "gene_name": "Whirlin"
}